{
  "term_id": "UNKNOWN:0003",
  "gene_symbol": "METTL27",
  "gene_name": "Methyltransferase-like protein 27",
  "gene": "UniProtKB:Q8N6F8",
  "term_label": "Unknown cellular component"
}